molybdate ion transmembrane transporter activity [GO:0015098] (molecular function) Also known as: molybdate transporter activity Subtypes: ABC-type molybdate transporter activity [GO:0015412] Definition: Enables the transfer of molybdate (MoO4 2-) ions from one side of a membrane to the other. Molybdate is the bivalent anion derived from molybdic acid. Relationships: is a type of transmembrane transporter activity [GO:0022857]; is part of molybdate ion transport [GO:0015689] Sources: ISBN:0198506732